histone H3-containing nucleosome [GO:0140573] (cellular component) Definition: A complex comprised of DNA wound around a multisubunit core and associated proteins containing the histone H3, which forms the primary packing unit of DNA into higher order structures. Relationships: is a type of nucleosome [GO:0000786] Also known as: histone H3 containing nucleosome References: PMID:33155135